{
  "term_label": "precatalytic spliceosome",
  "term_id": "GO:0071011",
  "gene_name": "U6 snRNA-associated Sm-like protein LSm2",
  "gene_symbol": "LSM2",
  "gene": "UniProtKB:Q9Y333"
}